{
  "gene": "UniProtKB:O60248",
  "term_id": "GO:0030182",
  "gene_symbol": "SOX15",
  "gene_name": "Protein SOX-15",
  "term_label": "neuron differentiation"
}